{
  "gene_name": "Mini-chromosome maintenance complex-binding protein",
  "gene_symbol": "MCMBP",
  "term_label": "DNA-templated DNA replication",
  "term_id": "GO:0006261",
  "gene": "UniProtKB:Q9BTE3"
}